{
  "gene_symbol": "SOD2",
  "gene_name": "Superoxide dismutase [Mn], mitochondrial",
  "term_label": "mitochondrion",
  "gene": "UniProtKB:P04179",
  "term_id": "GO:0005739"
}